{
  "gene_symbol": "CCR9",
  "term_id": "GO:0060326",
  "gene": "UniProtKB:P51686",
  "gene_name": "C-C chemokine receptor type 9",
  "term_label": "cell chemotaxis"
}